{
  "term_label": "Unknown cellular component",
  "term_id": "UNKNOWN:0003",
  "gene_symbol": "RASL10B",
  "gene": "UniProtKB:Q96S79",
  "gene_name": "Ras-like protein family member 10B"
}